negative regulation of establishment of protein-containing complex localization to telomere [GO:1904914] (biological process) References: PMID:26586433 Sources: GOC:BHF, GOC:BHF_telomere, GOC:TermGenie, GOC:rph, GO_REF:0000058 Definition: Any process that stops, prevents or reduces the frequency, rate or extent of establishment of the localization of a protein-containing macromolecular complex to a telomere. Also known as: down regulation of establishment of macromolecular complex localisation to telomere, down regulation of establishment of macromolecular complex localization to telomere, down-regulation of establishment of macromolecular complex localisation to telomere, down-regulation of establishment of macromolecular complex localization to telomere, downregulation of establishment of macromolecular complex localisation to telomere, downregulation of establishment of macromolecular complex localization to telomere, negative regulation of establishment of macromolecular complex localisation to telomere, inhibition of establishment of macromolecular complex localisation to telomere, inhibition of establishment of macromolecular complex localization to telomere, negative regulation of establishment of macromolecular complex localization to telomere Relationships: is a type of GO:0048519; is a type of regulation of establishment of protein-containing complex localization to telomere [GO:1904913]; negatively regulates establishment of protein-containing complex localization to telomere [GO:0097695]